{
  "gene": "UniProtKB:Q99807",
  "term_id": "GO:0005634",
  "gene_name": "5-demethoxyubiquinone hydroxylase, mitochondrial",
  "gene_symbol": "COQ7",
  "term_label": "nucleus"
}